gibberellin A9 carboxyl methyltransferase activity [GO:0102117] (molecular function) Sources: EC:2.1.1.275, GOC:pz Relationships: is a type of methyltransferase activity [GO:0008168] Definition: Catalysis of the reaction: gibberellin A9 + S-adenosyl-L-methionine = gibberellin A9 methyl ester + S-adenosyl-L-homocysteine.